{
  "gene_symbol": "MED21",
  "term_id": "GO:0016592",
  "gene_name": "Mediator of RNA polymerase II transcription subunit 21",
  "term_label": "mediator complex",
  "gene": "UniProtKB:Q13503"
}